GTP diphosphatase activity [GO:0036219] (molecular function) References: PMID:22531138 Sources: GOC:dgf, RHEA:29391 Relationships: is a type of nucleoside triphosphate diphosphatase activity [GO:0047429] Also known as: GTP diphosphohydrolase (diphosphate-forming); guanosine 5'-triphosphate pyrophosphohydrolase, GTP diphosphohydrolase activity, GTP pyrophosphatase activity Definition: Catalysis of the reaction: GTP + H2O = GMP + H+ + diphosphate.